{
  "term_label": "ATP hydrolysis activity",
  "gene": "UniProtKB:P33176",
  "term_id": "GO:0016887",
  "gene_name": "Kinesin-1 heavy chain",
  "gene_symbol": "KIF5B"
}